mitotic nuclear pore complex reassembly [GO:0007087] (biological process) Definition: The cell cycle process in which nuclear pore complexes reform during mitotic cell division. Sources: GOC:ai Relationships: is a type of GO:0051292; is a type of mitotic cell cycle process [GO:1903047]; BFO_0000050 mitotic nuclear membrane reassembly [GO:0007084]